inositol-4,5,6-triphosphate 5-phosphatase activity [GO:1990648] (molecular function) References: PMID:15316017 Sources: GOC:al Definition: Catalysis of the reaction: 1D-myo-inositol 4,5,6-trisphosphate + H2O = 1D-myo-inositol 4,6-bisphosphate + phosphate. Relationships: is a type of GO:0046030